{
  "gene_name": "Heat shock factor protein 5",
  "gene": "UniProtKB:Q4G112",
  "term_label": "RNA polymerase II cis-regulatory region sequence-specific DNA binding",
  "gene_symbol": "HSF5",
  "term_id": "GO:0000978"
}